{
  "gene_symbol": "CSNK1A1",
  "term_label": "protein serine/threonine kinase activity",
  "gene_name": "Casein kinase I isoform alpha",
  "gene": "UniProtKB:P48729",
  "term_id": "GO:0004674"
}